{
  "gene_symbol": "ZC3H18",
  "term_label": "Unknown molecular function",
  "term_id": "UNKNOWN:0001",
  "gene": "UniProtKB:Q86VM9",
  "gene_name": "Zinc finger CCCH domain-containing protein 18"
}